regulation of astrocyte chemotaxis [GO:2000458] (biological process) Definition: Any process that modulates the frequency, rate or extent of astrocyte chemotaxis. Sources: GOC:obol Relationships: is a type of GO:0050920; is a type of regulation of glial cell migration [GO:1903975]; regulates astrocyte chemotaxis [GO:0035700] Subtypes: negative regulation of astrocyte chemotaxis [GO:2000459], GO:2000464